{
  "term_id": "UNKNOWN:0003",
  "gene": "UniProtKB:Q9H7Y0",
  "term_label": "Unknown cellular component",
  "gene_name": "Divergent protein kinase domain 2B",
  "gene_symbol": "DIPK2B"
}